{
  "gene": "UniProtKB:O75592",
  "term_label": "nucleus",
  "gene_symbol": "MYCBP2",
  "gene_name": "E3 ubiquitin-protein ligase MYCBP2",
  "term_id": "GO:0005634"
}